{
  "term_label": "cytosol",
  "gene_symbol": "HSPA4L",
  "gene": "UniProtKB:O95757",
  "term_id": "GO:0005829",
  "gene_name": "Heat shock 70 kDa protein 4L"
}